{
  "term_id": "GO:0005759",
  "gene": "UniProtKB:Q53FZ2",
  "gene_symbol": "ACSM3",
  "gene_name": "Acyl-coenzyme A synthetase ACSM3, mitochondrial",
  "term_label": "mitochondrial matrix"
}